mitochondrial mRNA 3'-end processing [GO:0090616] (biological process) Definition: Any process involved in forming the mature 3' end of an mRNA molecule that derives from the mitochondrial genome. Relationships: is a type of mitochondrial RNA 3'-end processing [GO:0000965]; is a type of mRNA 3'-end processing [GO:0031124]; is_a GO:0090615 References: PMID:25181358 Sources: GOC:tb